{
  "gene_name": "Integrin beta-6",
  "gene_symbol": "ITGB6",
  "term_id": "GO:0098609",
  "term_label": "cell-cell adhesion",
  "gene": "UniProtKB:P18564"
}